{
  "gene_symbol": "RAD51B",
  "gene_name": "DNA repair protein RAD51 homolog 2",
  "term_label": "Rad51B-Rad51C-Rad51D-XRCC2 complex",
  "gene": "UniProtKB:O15315",
  "term_id": "GO:0033063"
}